IMP cyclohydrolase activity [GO:0003937] (molecular function) Sources: EC:3.5.4.10 Definition: Catalysis of the reaction: IMP + H2O = 5-formamido-1-(5-phosphoribosyl)imidazole-4-carboxamide. Relationships: is a type of cyclohydrolase activity [GO:0019238] Also known as: IMP 1,2-hydrolase (decyclizing), IMP synthetase activity, inosinate cyclohydrolase activity, inosinicase activity